6-sulfoquinovose(1-) catabolic process to glycerone phosphate and 3-sulfolactaldehyde [GO:0061720] (biological process) References: PMID:24463506 Sources: GOC:dph Definition: The chemical reactions and pathways resulting in the breakdown of 6-sulfoquinovose(1-) resulting in the formation of glycerone phosphate (DHAP) and 3-sulfolactaldehyde (SLA). Relationships: is_a aldehyde metabolic process [GO:0006081]; is a type of phosphate-containing compound metabolic process [GO:0006796]; is a type of organophosphate metabolic process [GO:0019637]; is a type of GO:0019694; is a type of primary alcohol metabolic process [GO:0034308]; is a type of ketone metabolic process [GO:0042180]; is a type of GO:1902652; is a type of 6-sulfoquinovose(1-) catabolic process [GO:1902777]; has part GO:0061593; has part 6-deoxy-6-sulfofructose kinase activity [GO:0061594]; has part 6-deoxy-6-sulfofructose-1-phosphate aldolase activity [GO:0061595]